SCF-Ctf13 ubiquitin ligase complex [GO:0097661] (cellular component) Definition: An SCF ubiquitin ligase complex in which the F-box protein is Ctf13 in S. cerevisiae. Relationships: is a type of SCF ubiquitin ligase complex [GO:0019005] References: PMID:14747994 Sources: GOC:jd, GOC:vw